{
  "term_label": "zymogen activation",
  "term_id": "GO:0031638",
  "gene": "UniProtKB:P00748",
  "gene_name": "Coagulation factor XII",
  "gene_symbol": "F12"
}